{
  "term_id": "GO:0000981",
  "gene_symbol": "ZNF396",
  "gene_name": "Zinc finger protein 396",
  "gene": "UniProtKB:Q96N95",
  "term_label": "DNA-binding transcription factor activity, RNA polymerase II-specific"
}